{
  "gene_name": "Thyroid hormone receptor alpha",
  "term_label": "thyroid hormone receptor signaling pathway",
  "term_id": "GO:0002154",
  "gene": "UniProtKB:P10827",
  "gene_symbol": "THRA"
}